{
  "term_id": "GO:0031167",
  "gene_name": "rRNA N6-adenosine-methyltransferase ZCCHC4",
  "gene_symbol": "ZCCHC4",
  "gene": "UniProtKB:Q9H5U6",
  "term_label": "rRNA methylation"
}